{
  "gene": "UniProtKB:Q9NXK6",
  "term_label": "Unknown cellular component",
  "gene_symbol": "PAQR5",
  "term_id": "UNKNOWN:0003",
  "gene_name": "Membrane progestin receptor gamma"
}